{
  "gene_symbol": "OPRD1",
  "term_id": "GO:0042923",
  "gene_name": "Delta-type opioid receptor",
  "term_label": "neuropeptide binding",
  "gene": "UniProtKB:P41143"
}